regulation of chronic inflammatory response to antigenic stimulus [GO:0002874] (biological process) Sources: GOC:add Subtypes: negative regulation of chronic inflammatory response to antigenic stimulus [GO:0002875], positive regulation of chronic inflammatory response to antigenic stimulus [GO:0002876] Definition: Any process that modulates the frequency, rate, or extent of a chronic inflammatory response to an antigenic stimulus. Relationships: is a type of regulation of chronic inflammatory response [GO:0002676]; is a type of regulation of inflammatory response to antigenic stimulus [GO:0002861]; regulates chronic inflammatory response to antigenic stimulus [GO:0002439]